{
  "term_id": "UNKNOWN:0001",
  "gene_symbol": "TMEM132E-DT",
  "gene_name": "Uncharacterized protein TMEM132E-DT",
  "term_label": "Unknown molecular function",
  "gene": "UniProtKB:A2RUQ5"
}